{
  "gene_symbol": "SYNPO2",
  "term_id": "GO:0030018",
  "term_label": "Z disc",
  "gene_name": "Synaptopodin-2",
  "gene": "UniProtKB:Q9UMS6"
}